{
  "gene_symbol": "OSBPL10",
  "gene_name": "Oxysterol-binding protein-related protein 10",
  "term_label": "cholesterol binding",
  "term_id": "GO:0015485",
  "gene": "UniProtKB:Q9BXB5"
}